regulation of cold-induced thermogenesis [GO:0120161] (BP) References: PMID:27876809 Also known as: regulation of CIT Relationships: is a type of GO:0019222; is a type of regulation of multicellular organismal process [GO:0051239]; regulates GO:0106106 Definition: Any process that modulates the frequency, rate or extent of cold-induced thermogenesis. Subtypes: positive regulation of cold-induced thermogenesis [GO:0120162], GO:0120163